{
  "gene": "UniProtKB:Q9NV56",
  "gene_name": "MRG_MORF4L-binding protein",
  "term_id": "GO:0006357",
  "term_label": "regulation of transcription by RNA polymerase II",
  "gene_symbol": "MRGBP"
}